negative regulation of proteolysis involved in protein catabolic process [GO:1903051] (biological process) Relationships: is a type of negative regulation of proteolysis [GO:0045861]; is a type of regulation of proteolysis involved in protein catabolic process [GO:1903050]; RO_0002212 proteolysis involved in protein catabolic process [GO:0051603] Also known as: down regulation of peptidolysis involved in cellular protein catabolic process, down regulation of peptidolysis involved in cellular protein catabolism, down regulation of proteolysis involved in cellular protein catabolic process, down-regulation of peptidolysis involved in cellular protein catabolic process, down-regulation of peptidolysis involved in cellular protein catabolism, down-regulation of proteolysis involved in cellular protein catabolic process, downregulation of peptidolysis involved in cellular protein catabolic process, downregulation of peptidolysis involved in cellular protein catabolism, downregulation of proteolysis involved in cellular protein catabolic process, negative regulation of peptidolysis involved in cellular protein catabolic process, negative regulation of peptidolysis involved in cellular protein catabolism, negative regulation of proteolysis involved in cellular protein catabolic process, inhibition of peptidolysis involved in cellular protein catabolic process, inhibition of peptidolysis involved in cellular protein catabolism, inhibition of proteolysis involved in cellular protein catabolic process, down regulation of peptidolysis during cellular protein catabolic process, down regulation of peptidolysis during cellular protein catabolism, down regulation of proteolysis during cellular protein catabolic process, down regulation of proteolysis during cellular protein catabolism, down-regulation of peptidolysis during cellular protein catabolic process, down-regulation of peptidolysis during cellular protein catabolism, down-regulation of proteolysis during cellular protein catabolic process, down-regulation of proteolysis during cellular protein catabolism, downregulation of peptidolysis during cellular protein catabolic process, downregulation of peptidolysis during cellular protein catabolism, downregulation of proteolysis during cellular protein catabolic process, downregulation of proteolysis during cellular protein catabolism, inhibition of peptidolysis during cellular protein catabolic process, inhibition of peptidolysis during cellular protein catabolism, inhibition of proteolysis during cellular protein catabolic process, inhibition of proteolysis during cellular protein catabolism, negative regulation of peptidolysis during cellular protein catabolic process, negative regulation of peptidolysis during cellular protein catabolism, negative regulation of proteolysis during cellular protein catabolic process, negative regulation of proteolysis during cellular protein catabolism Subtypes: negative regulation of proteolysis associated with antigen processing and presentation [GO:0002629], GO:1901799, negative regulation of ubiquitin-dependent protein catabolic process [GO:2000059] References: PMID:18307834 Sources: GOC:BHF, GOC:TermGenie, GOC:rl, GO_REF:0000058 Definition: Any process that stops, prevents or reduces the frequency, rate or extent of proteolysis involved in protein catabolic process. Note: Overexpression of cathepsin C propeptide significantly increased the degradation of intestinal alkaline phosphatase (IAP).